chronic inflammatory response [GO:0002544] (biological process) Regulation: regulated by GO:0002676; negatively regulated by negative regulation of chronic inflammatory response [GO:0002677]; positively regulated by positive regulation of chronic inflammatory response [GO:0002678] Relationships: is a type of inflammatory response [GO:0006954] Definition: Inflammation of prolonged duration (weeks or months) in which active inflammation, tissue destruction, and attempts at repair are proceeding simultaneously. Although it may follow acute inflammation, chronic inflammation frequently begins insidiously, as a low-grade, smoldering, often asymptomatic response. Subtypes: chronic inflammatory response to antigenic stimulus [GO:0002439], GO:0002545 Sources: GOC:jal, GO_REF:0000022, ISBN:0781735149